{
  "term_label": "90S preribosome",
  "term_id": "GO:0030686",
  "gene_name": "Ribosome biogenesis protein BMS1 homolog",
  "gene_symbol": "BMS1",
  "gene": "UniProtKB:Q14692"
}